{
  "gene_name": "Hypoxia-inducible factor 3-alpha",
  "term_id": "GO:0006357",
  "gene": "UniProtKB:Q9Y2N7",
  "term_label": "regulation of transcription by RNA polymerase II",
  "gene_symbol": "HIF3A"
}